{
  "gene_name": "Splicing factor U2AF 35 kDa subunit",
  "term_label": "pre-mRNA 3'-splice site binding",
  "gene_symbol": "U2AF1",
  "term_id": "GO:0030628",
  "gene": "UniProtKB:Q01081"
}